response to hexose [GO:0009746] (biological process) Also known as: response to hexose stimulus Subtypes: GO:0009732, response to glucose [GO:0009749], response to fructose [GO:0009750], response to rhamnose [GO:0032149], GO:0071331, response to D-galactose [GO:1905377], response to mannose [GO:1905582] Relationships: is_a response to monosaccharide [GO:0034284] Sources: GOC:jl Definition: Any process that results in a change in state or activity of a cell or an organism (in terms of movement, secretion, enzyme production, gene expression, etc.) as a result of a hexose stimulus.